{
  "gene": "UniProtKB:Q8N2E2",
  "term_id": "UNKNOWN:0002",
  "gene_symbol": "VWDE",
  "gene_name": "von Willebrand factor D and EGF domain-containing protein",
  "term_label": "Unknown biological process"
}